{
  "gene_symbol": "SRCAP",
  "gene_name": "Helicase SRCAP",
  "gene": "UniProtKB:Q6ZRS2",
  "term_label": "histone binding",
  "term_id": "GO:0042393"
}